{
  "term_id": "GO:0000981",
  "gene_name": "Forkhead box protein E1",
  "gene_symbol": "FOXE1",
  "gene": "UniProtKB:O00358",
  "term_label": "DNA-binding transcription factor activity, RNA polymerase II-specific"
}